xanthosine:proton symporter activity [GO:0015537] (molecular function) Definition: Enables the transfer of a solute or solutes from one side of a membrane to the other according to the reaction: xanthosine(out) + H+(out) = xanthosine(in) + H+(in). Also known as: xanthosine:hydrogen ion symporter activity, xanthosine permease activity Relationships: is a type of GO:0015506; is a type of xanthosine transmembrane transporter activity [GO:0015553] Sources: TC:2.A.1.10.2